tube viral factory [GO:0039719] (cellular component) Relationships: is a type of cytoplasmic viral factory [GO:0039714] Sources: VZ:1951 Definition: A cytoplasmic viral factory derived from the Golgi in which Bunyaviridae replication takes place. Tubes are membranous structures close to the assembly and budding sites, and their function may be to connect viral replication and morphogenesis inside viral factories.